{
  "term_label": "glutathione transferase activity",
  "gene_name": "Glutathione S-transferase theta-1",
  "gene_symbol": "GSTT1",
  "gene": "UniProtKB:P30711",
  "term_id": "GO:0004364"
}